{
  "term_label": "extrinsic component of presynaptic endocytic zone membrane",
  "gene_symbol": "SNAP91",
  "gene_name": "Clathrin coat assembly protein AP180",
  "term_id": "GO:0098894",
  "gene": "UniProtKB:O60641"
}